{
  "gene_symbol": "RAB29",
  "term_id": "GO:0003924",
  "term_label": "GTPase activity",
  "gene_name": "Ras-related protein Rab-7L1",
  "gene": "UniProtKB:O14966"
}